{
  "gene": "UniProtKB:Q15027",
  "term_label": "Unknown biological process",
  "gene_name": "Arf-GAP with coiled-coil, ANK repeat and PH domain-containing protein 1",
  "term_id": "UNKNOWN:0002",
  "gene_symbol": "ACAP1"
}